{
  "gene_name": "Vacuolar protein sorting-associated protein 37C",
  "gene_symbol": "VPS37C",
  "term_id": "GO:0043162",
  "gene": "UniProtKB:A5D8V6",
  "term_label": "ubiquitin-dependent protein catabolic process via the multivesicular body sorting pathway"
}